rough endoplasmic reticulum lumen [GO:0048237] (cellular component) Relationships: is a type of endoplasmic reticulum lumen [GO:0005788]; is part of GO:0005791 Also known as: RER lumen, rough ER lumen Sources: GOC:jid Definition: The volume enclosed by the membranes of the rough endoplasmic reticulum.